ribosomal small subunit biogenesis [GO:0042274] (biological process) Relationships: is a type of ribonucleoprotein complex biogenesis [GO:0022613]; is part of ribosome biogenesis [GO:0042254] Sources: GOC:jl Definition: A cellular process that results in the biosynthesis of constituent macromolecules, assembly, and arrangement of constituent parts of a small ribosomal subunit; includes transport to the sites of protein synthesis. Also known as: ribosomal small subunit biogenesis and assembly